{
  "gene": "UniProtKB:P07315",
  "term_id": "GO:0002088",
  "gene_symbol": "CRYGC",
  "term_label": "lens development in camera-type eye",
  "gene_name": "Gamma-crystallin C"
}